cellular response to 1-oleoyl-sn-glycerol 3-phosphate [GO:1904566] (biological process) Also known as: cellular response to 1-oleoyl lysophosphatidic acid, cellular response to LPA, cellular response to lysophosphatidic acid, cellular response to oleoyl lysophosphatidic acid, cellular response to oleoyl-L-alpha-lysophosphatidic acid References: PMID:12139919 Sources: GOC:TermGenie, GO_REF:0000071 Relationships: is a type of cellular response to lipid [GO:0071396]; is_a cellular response to oxygen-containing compound [GO:1901701]; is a type of response to 1-oleoyl-sn-glycerol 3-phosphate [GO:1904565] Definition: Any process that results in a change in state or activity of a cell (in terms of movement, secretion, enzyme production, gene expression, etc.) as a result of a 1-oleoyl-sn-glycerol 3-phosphate stimulus.